{
  "gene_name": "ATP synthase subunit ATP5MJ, mitochondrial",
  "gene": "UniProtKB:P56378",
  "gene_symbol": "ATP5MJ",
  "term_id": "GO:0045259",
  "term_label": "proton-transporting ATP synthase complex"
}